(+)-epi-alpha-bisabolol biosynthetic process [GO:1901943] (biological process) Relationships: is a type of sesquiterpenoid biosynthetic process [GO:0016106] Definition: The chemical reactions and pathways resulting in the formation of (+)-epi-alpha-bisabolol. Also known as: (+)-epi-alpha-bisabolol anabolism, (+)-epi-alpha-bisabolol biosynthesis, (+)-epi-alpha-bisabolol formation, (+)-epi-alpha-bisabolol synthesis References: PMID:22867794 Sources: GOC:TermGenie